{
  "gene_name": "Proteasome subunit alpha type-1",
  "gene": "UniProtKB:P25786",
  "term_id": "UNKNOWN:0001",
  "term_label": "Unknown molecular function",
  "gene_symbol": "PSMA1"
}